{
  "gene_name": "Coatomer subunit gamma-1",
  "gene": "UniProtKB:Q9Y678",
  "gene_symbol": "COPG1",
  "term_id": "GO:0009306",
  "term_label": "protein secretion"
}